{
  "gene_symbol": "OLFML1",
  "gene": "UniProtKB:Q6UWY5",
  "gene_name": "Olfactomedin-like protein 1",
  "term_label": "extracellular space",
  "term_id": "GO:0005615"
}